{
  "gene": "UniProtKB:Q9UP95",
  "gene_name": "Solute carrier family 12 member 4",
  "term_label": "potassium ion homeostasis",
  "gene_symbol": "SLC12A4",
  "term_id": "GO:0055075"
}